rRNA methyltransferase activity [GO:0008649] (molecular function) Sources: GOC:mah Subtypes: rRNA (adenine) methyltransferase activity [GO:0016433], rRNA (cytosine) methyltransferase activity [GO:0016434], GO:0016435, GO:0016436, rRNA (pseudouridine) methyltransferase activity [GO:0070037] Definition: Catalysis of the transfer of a methyl group from S-adenosyl-L-methionine to a nucleoside residue in an rRNA molecule. Relationships: is a type of RNA methyltransferase activity [GO:0008173]; is a type of S-adenosylmethionine-dependent methyltransferase activity [GO:0008757]; is a type of catalytic activity, acting on a rRNA [GO:0140102]; is part of rRNA methylation [GO:0031167]